protein kinase C inhibitor activity [GO:0008426] (molecular function) Sources: GOC:ai Relationships: is a type of protein serine/threonine kinase inhibitor activity [GO:0030291]; negatively regulates diacylglycerol-dependent serine/threonine kinase activity [GO:0004697] Definition: Binds to and stops, prevents or reduces the activity of protein kinase C, an enzyme which phosphorylates a protein. Also known as: PKC inhibitor activity, diacylglycerol-activated phospholipid-dependent PKC inhibitor activity, diacylglycerol-activated phospholipid-dependent protein kinase C inhibitor activity